{
  "gene_symbol": "CELA2A",
  "term_id": "GO:1901143",
  "gene": "UniProtKB:P08217",
  "term_label": "insulin catabolic process",
  "gene_name": "Chymotrypsin-like elastase family member 2A"
}